regulation of acetylcholine uptake [GO:0051631] (biological process) Definition: Any process that modulates the frequency, rate or extent of the directed movement of the neurotransmitter acetylcholine into a cell. Sources: GOC:ai Subtypes: GO:0051632, GO:0051633 Also known as: regulation of acetylcholine import Relationships: is a type of regulation of amine transport [GO:0051952]; regulates GO:0051630